aggrephagy [GO:0035973] (biological process) Relationships: is a type of macroautophagy [GO:0016236] Regulation: regulated by GO:1905335; RO_0002212 by negative regulation of aggrephagy [GO:1905336]; positively regulated by positive regulation of aggrephagy [GO:1905337] References: PMID:18508269, PMID:25062811 Sources: GOC:autophagy, GOC:kmv Definition: The selective degradation of protein aggregates by macroautophagy.